{
  "gene_name": "Inositol-trisphosphate 3-kinase A",
  "term_id": "GO:0046854",
  "gene_symbol": "ITPKA",
  "gene": "UniProtKB:P23677",
  "term_label": "phosphatidylinositol phosphate biosynthetic process"
}